IkappaB kinase activity [GO:0008384] (molecular function) Definition: Catalysis of the reaction: ATP + IkappaB protein = ADP + IkappaB phosphoprotein. Relationships: is a type of GO:0004674; is part of I-kappaB phosphorylation [GO:0007252] Also known as: TANK-binding kinase 1 activity, ATP:IkappaB protein phosphotransferase activity, CHUK, IKBKA, IKBKB, IKK, IKK-1, IKK-2, STK12, TBK1, inhibitor of NF-kappaB kinase activity, inhibitor of NFkappaB kinase activity Note: Note that phosphorylation of IkappaB targets it for proteasomal degradation and allows the nuclear translocation of kB. Sources: EC:2.7.11.10